{
  "gene_symbol": "OR4X1",
  "gene_name": "Olfactory receptor 4X1",
  "gene": "UniProtKB:Q8NH49",
  "term_id": "GO:0004984",
  "term_label": "olfactory receptor activity"
}